{
  "gene": "UniProtKB:Q15018",
  "gene_name": "BRISC complex subunit Abraxas 2",
  "term_label": "polyubiquitin modification-dependent protein binding",
  "gene_symbol": "ABRAXAS2",
  "term_id": "GO:0031593"
}